{
  "term_id": "GO:0051015",
  "gene_name": "Myosin-8",
  "gene_symbol": "MYH8",
  "gene": "UniProtKB:P13535",
  "term_label": "actin filament binding"
}